FtsZ-dependent cytokinesis [GO:0043093] (BP) Also known as: cytokinesis by binary fission, prokaryote-type cytokinesis, prokaryotic fission Definition: A cytokinesis process that involves a set of conserved proteins including FtsZ, and results in the formation of two similarly sized and shaped cells. Regulation: regulated by regulation of FtsZ-dependent cytokinesis [GO:2000244]; negatively regulated by negative regulation of FtsZ-dependent cytokinesis [GO:2000245]; positively regulated by positive regulation of FtsZ-dependent cytokinesis [GO:2000246] Note: Note that this term is intended for the annotation of prokaryotic gene products. References: PMID:12626683 Sources: GOC:mah, ISBN:0815108893 Relationships: is a type of GO:0000910; is a type of reproductive process in single-celled organism [GO:0022413]; is part of asexual reproduction [GO:0019954]